{
  "gene_symbol": "PEX26",
  "gene_name": "Peroxisome assembly protein 26",
  "gene": "UniProtKB:Q7Z412",
  "term_id": "GO:0051117",
  "term_label": "ATPase binding"
}